{
  "term_id": "GO:0030308",
  "gene_symbol": "OSGIN1",
  "term_label": "negative regulation of cell growth",
  "gene": "UniProtKB:Q9UJX0",
  "gene_name": "Oxidative stress-induced growth inhibitor 1"
}